{
  "gene_name": "tRNA-dihydrouridine(16_17) synthase [NAD(P)(+)]-like",
  "gene_symbol": "DUS1L",
  "term_label": "Unknown biological process",
  "gene": "UniProtKB:Q6P1R4",
  "term_id": "UNKNOWN:0002"
}